{
  "gene_name": "Putative STAG3-like protein 4",
  "term_label": "Unknown biological process",
  "gene": "UniProtKB:Q8TBR4",
  "gene_symbol": "STAG3L4",
  "term_id": "UNKNOWN:0002"
}